{
  "term_label": "release of sequestered calcium ion into cytosol by sarcoplasmic reticulum",
  "gene": "UniProtKB:Q13061",
  "term_id": "GO:0014808",
  "gene_name": "Triadin",
  "gene_symbol": "TRDN"
}